{
  "gene": "UniProtKB:Q9NTI7",
  "gene_symbol": "INKA2",
  "term_id": "GO:0030291",
  "term_label": "protein serine/threonine kinase inhibitor activity",
  "gene_name": "PAK4-inhibitor INKA2"
}